endosomal lumen acidification [GO:0048388] (biological process) Definition: Any process that reduces the pH of the endosomal lumen, measured by the concentration of the hydrogen ion. Relationships: is a type of intracellular pH reduction [GO:0051452]; is part of endosome organization [GO:0007032] Sources: GOC:jid